{
  "gene_name": "GTP-binding protein SAR1b",
  "gene_symbol": "SAR1B",
  "term_label": "vesicle organization",
  "term_id": "GO:0016050",
  "gene": "UniProtKB:Q9Y6B6"
}